{
  "gene_symbol": "ACTN3",
  "term_label": "cortical actin cytoskeleton",
  "gene": "UniProtKB:Q08043",
  "term_id": "GO:0030864",
  "gene_name": "Alpha-actinin-3"
}